{
  "gene_name": "Lactosylceramide 4-alpha-galactosyltransferase",
  "gene": "UniProtKB:Q9NPC4",
  "gene_symbol": "A4GALT",
  "term_label": "glycosphingolipid biosynthetic process",
  "term_id": "GO:0006688"
}